mitochondrial electron transport, ubiquinol to cytochrome c [GO:0006122] (biological process) Definition: The transfer of electrons from ubiquinol to cytochrome c that occurs during oxidative phosphorylation, mediated by the multisubunit enzyme known as complex III. Also known as: complex III (ubiquinone to cytochrome c) Relationships: is a type of GO:0019646; is part of mitochondrial ATP synthesis coupled electron transport [GO:0042775] Sources: ISBN:0716731363